nuclear migration along microfilament [GO:0031022] (biological process) Sources: GOC:mah Definition: The directed movement of the nucleus along microfilaments within the cell, mediated by motor proteins. Relationships: is a type of nuclear migration [GO:0007097]; is a type of actin filament-based movement [GO:0030048]; is_a actin filament-based transport [GO:0099515] Also known as: nuclear migration, microfilament-mediated